negative regulation of developmental process [GO:0051093] (BP) Definition: Any process that stops, prevents or reduces the rate or extent of development, the biological process whose specific outcome is the progression of an organism over time from an initial condition (e.g. a zygote, or a young adult) to a later condition (e.g. a multicellular animal or an aged adult). Sources: GOC:ai Also known as: down regulation of developmental process, down-regulation of developmental process, downregulation of developmental process, inhibition of developmental process Relationships: is a type of negative regulation of biological process [GO:0048519]; is a type of GO:0050793; negatively regulates developmental process [GO:0032502] Subtypes: negative regulation of germinal center formation [GO:0002635], GO:0002644, negative regulation of Wnt signaling pathway involved in heart development [GO:0003308], negative regulation of mitochondrial fusion [GO:0010637], GO:0031495, GO:0034242, GO:0043939, negative regulation of cell differentiation [GO:0045596], negative regulation of epidermis development [GO:0045683], negative regulation of salivary gland boundary specification [GO:0045705], negative regulation of chitin-based cuticle tanning [GO:0045800], GO:0045804, negative regulation of isotype switching [GO:0045829], negative regulation of embryonic development [GO:0045992], negative regulation of retinal cell programmed cell death [GO:0046671], negative regulation of cuticle pigmentation [GO:0048080], negative regulation of female pigmentation [GO:0048090], GO:0048092, negative regulation of post-embryonic development [GO:0048581], GO:0048635, negative regulation of developmental growth [GO:0048640], negative regulation of hair follicle development [GO:0051799], GO:0051961, GO:0060313, negative regulation of epithelial cell proliferation involved in prostate gland development [GO:0060770], GO:0060862, GO:0061000, GO:0061037, negative regulation of entry into reproductive diapause [GO:0061964], negative regulation of somatic muscle development [GO:0062225], GO:0070168, GO:0070571, negative regulation of conidiophore stalk development [GO:0070800], GO:0072200, negative regulation of germ tube formation [GO:0075012], GO:0075019, negative regulation of formation of symbiont germ tube hook structure for appressorium development [GO:0075032], negative regulation of infection cushion formation [GO:0075186], negative regulation of hyphopodium formation [GO:0075190], negative regulation of haustorium mother cell formation [GO:0075195], GO:0075262, negative regulation of kidney development [GO:0090185], negative regulation of mitochondrial fission [GO:0090258], negative regulation of aggregation involved in sorocarp development [GO:0110014], negative regulation of nematode male tail tip morphogenesis [GO:0110038], GO:0110081, negative regulation of animal organ morphogenesis [GO:0110111], negative regulation of imaginal disc-derived leg joint morphogenesis [GO:0110139], negative regulation of pre-B cell receptor expression [GO:0140646], negative regulation of neuron projection arborization [GO:0150013], negative regulation of leaf senescence [GO:1900056], negative regulation of bone trabecula formation [GO:1900155], negative regulation of pronephric nephron tubule development [GO:1900207], negative regulation of cardiac chamber formation [GO:1901211], negative regulation of cardiac chamber morphogenesis [GO:1901220], negative regulation of heart induction [GO:1901320], negative regulation of vasculature development [GO:1901343], negative regulation of lymphangiogenesis [GO:1901491], negative regulation of synaptic vesicle lumen acidification [GO:1901547], GO:1901862, negative regulation of sclerotium development [GO:1901923], negative regulation of seed dormancy process [GO:1902039], GO:1902184, negative regulation of stem cell population maintenance [GO:1902455], negative regulation of embryonic skeletal joint development [GO:1902763], GO:1902864, negative regulation of retina development in camera-type eye [GO:1902867], GO:1903011, negative regulation of tube lumen cavitation [GO:1903133], negative regulation of lactation [GO:1903488], negative regulation of endosperm development [GO:1904095], negative regulation of adipose tissue development [GO:1904178], negative regulation of age-related resistance [GO:1904249], negative regulation of basement membrane assembly involved in embryonic body morphogenesis [GO:1904260], GO:1904360, negative regulation of cardiac ventricle development [GO:1904413], negative regulation of thyroid gland epithelial cell proliferation [GO:1904442], negative regulation of lung alveolus development [GO:1904654], GO:1904746, negative regulation of apical ectodermal ridge formation [GO:1905141], GO:1905175, negative regulation of morphogenesis of an epithelium [GO:1905331], negative regulation of plant organ morphogenesis [GO:1905422], GO:1905622, negative regulation of gonad development [GO:1905940], negative regulation of metanephric S-shaped body morphogenesis [GO:2000005], negative regulation of metanephric comma-shaped body morphogenesis [GO:2000007], negative regulation of mammary stem cell proliferation [GO:2000102], GO:2000171, negative regulation of branching morphogenesis of a nerve [GO:2000173], negative regulation of synapse maturation [GO:2000297], negative regulation of fibroblast growth factor receptor signaling pathway involved in neural plate anterior/posterior pattern formation [GO:2000314], negative regulation of blood microparticle formation [GO:2000333], negative regulation of ovarian follicle development [GO:2000355], negative regulation of mesoderm development [GO:2000381], negative regulation of ectoderm development [GO:2000384], negative regulation of lamellipodium morphogenesis [GO:2000393], negative regulation of optic nerve formation [GO:2000596], negative regulation of seed maturation [GO:2000692], negative regulation of anterior head development [GO:2000743], negative regulation of mesenchymal cell proliferation involved in lung development [GO:2000791], negative regulation of metanephric ureteric bud development [GO:2001075]